{
  "gene_name": "Mannan-binding lectin serine protease 2",
  "gene": "UniProtKB:O00187",
  "term_id": "GO:0004252",
  "term_label": "serine-type endopeptidase activity",
  "gene_symbol": "MASP2"
}